{
  "gene_name": "Metalloprotease TIKI1",
  "term_id": "GO:0016020",
  "gene_symbol": "TRABD2A",
  "term_label": "membrane",
  "gene": "UniProtKB:Q86V40"
}